regulation of cellular process [GO:0050794] (BP) Relationships: is a type of GO:0050789; regulates cellular process [GO:0009987] Sources: GOC:go_curators Also known as: regulation of cellular physiological process Subtypes: regulation of membrane depolarization [GO:0003254], signal transduction [GO:0007165], regulation of stomatal movement [GO:0010119], regulation of cell fate commitment [GO:0010453], regulation of septum digestion after cytokinesis [GO:0010590], regulation of cell communication [GO:0010646], regulation of lipid storage [GO:0010883], GO:0019222, regulation of cell adhesion [GO:0030155], regulation of cell killing [GO:0031341], regulation of myelination [GO:0031641], regulation of establishment or maintenance of cell polarity [GO:0032878], regulation of microtubule-based process [GO:0032886], regulation of actin filament-based process [GO:0032970], GO:0034762, regulation of cell population proliferation [GO:0042127], regulation of cytolysis [GO:0042268], GO:0043067, regulation of cellular component biogenesis [GO:0044087], GO:0045304, GO:0045595, positive regulation of cellular process [GO:0048522], GO:0048523, regulation of cell activation [GO:0050865], GO:0051128, regulation of sequestering of calcium ion [GO:0051282], regulation of cell division [GO:0051302], regulation of cell cycle [GO:0051726], regulation of cellular localization [GO:0060341], regulation of cell adhesion molecule production [GO:0060353], regulation of vesicle-mediated transport [GO:0060627], regulation of cellular response to stress [GO:0080135], regulation of vesicle docking [GO:0106020], regulation of cellular response to alkaline pH [GO:1900067], GO:1900076, regulation of execution phase of apoptosis [GO:1900117], regulation of single-species biofilm formation [GO:1900190], GO:1900239, GO:1902026, regulation of response to cell cycle checkpoint signaling [GO:1902145], regulation of synaptic vesicle transport [GO:1902803], regulation of horizontal cell localization [GO:1902872], GO:1902908, regulation of opsonization [GO:1903027], GO:1903332, GO:1903338, regulation of secretion by cell [GO:1903530], regulation of spore germination [GO:1904359], regulation of vascular associated smooth muscle cell dedifferentiation [GO:1905174], regulation of cellular response to manganese ion [GO:1905802], regulation of cellular response to gamma radiation [GO:1905843], regulation of cellular response to oxidopamine [GO:1905846], GO:1905890, GO:1905933, GO:1905957, regulation of cell motility [GO:2000145], GO:2000359, regulation of cellular response to testosterone stimulus [GO:2000654], regulation of cellular response to X-ray [GO:2000683], GO:2000772, GO:2001038 Definition: Any process that modulates the frequency, rate or extent of a cellular process, any of those that are carried out at the cellular level, but are not necessarily restricted to a single cell. For example, cell communication occurs among more than one cell, but occurs at the cellular level.